transketolase or transaldolase activity [GO:0016744] (molecular function) Relationships: is a type of transferase activity [GO:0016740] Also known as: transferase activity, transferring aldehyde or ketonic groups Definition: Catalysis of the transfer of an aldehyde or ketonic group from one compound (donor) to another (acceptor). Subtypes: acetolactate synthase activity [GO:0003984], GO:0004801, transketolase activity [GO:0004802], 1-deoxy-D-xylulose-5-phosphate synthase activity [GO:0008661], macrophomate synthase activity [GO:0033191], GO:0033806, acetoin-ribose-5-phosphate transaldolase activity [GO:0047156], GO:0047896, GO:0050439, 2-succinyl-5-enolpyruvyl-6-hydroxy-3-cyclohexene-1-carboxylic-acid synthase activity [GO:0070204] Sources: GOC:jl, ISBN:0198506732